{
  "term_label": "peptide antigen binding",
  "gene_symbol": "HLA-H",
  "term_id": "GO:0042605",
  "gene": "UniProtKB:P01893",
  "gene_name": "Putative HLA class I histocompatibility antigen, alpha chain H"
}